{
  "term_label": "cell differentiation",
  "gene_symbol": "VDR",
  "gene_name": "Vitamin D3 receptor",
  "term_id": "GO:0030154",
  "gene": "UniProtKB:P11473"
}